{
  "gene": "UniProtKB:A0A0J9YVP9",
  "term_id": "UNKNOWN:0003",
  "term_label": "Unknown cellular component",
  "gene_symbol": "IGHJ5",
  "gene_name": "Immunoglobulin heavy joining 5 (Fragment)"
}